subapical complex [GO:0035003] (cellular component) References: PMID:11752566, PMID:12500938 Definition: The most apical region of the lateral plasma membrane of an invertebrate epithelial cell. The subapical complex lies above the zonula adherens and the septate junction, and is comparable to the position of the tight junction of vertebrate cells. Also known as: SAC Relationships: is a type of plasma membrane protein complex [GO:0098797]; is part of apical junction complex [GO:0043296]